{
  "gene_symbol": "CCDC28B",
  "gene": "UniProtKB:Q9BUN5",
  "gene_name": "Coiled-coil domain-containing protein 28B",
  "term_label": "Unknown molecular function",
  "term_id": "UNKNOWN:0001"
}